{
  "gene_name": "N-acetylmuramoyl-L-alanine amidase",
  "term_label": "extracellular space",
  "gene_symbol": "PGLYRP2",
  "term_id": "GO:0005615",
  "gene": "UniProtKB:Q96PD5"
}